mycothiol-dependent detoxification [GO:0010127] (biological process) Also known as: mycothiol-dependent detoxification of alkylating agent Sources: GOC:pz Relationships: is_a GO:0098754 Definition: The chemical reactions using mycothiol to convert an alkylating agent to an S-conjugate of mycothiol. The latter is cleaved to release mercapturic acid which is excreted from the cell.